{
  "gene": "UniProtKB:Q14839",
  "term_label": "chromatin",
  "gene_name": "Chromodomain-helicase-DNA-binding protein 4",
  "term_id": "GO:0000785",
  "gene_symbol": "CHD4"
}